{
  "term_id": "GO:0000978",
  "term_label": "RNA polymerase II cis-regulatory region sequence-specific DNA binding",
  "gene_name": "Zinc finger protein 83",
  "gene": "UniProtKB:P51522",
  "gene_symbol": "ZNF83"
}